negative regulation of bile acid secretion [GO:0120190] (biological process) Definition: Any process that stops, prevents or reduces the frequency, rate or extent of the controlled release of bile acid from a cell or a tissue. References: PMID:22767443 Sources: GOC:BHF, GOC:BHF_miRNA, GOC:rph Relationships: is a type of GO:0032891; is a type of GO:0051048; is a type of GO:0120188; negatively regulates GO:0032782